vascular endothelial growth factor receptor 3 binding [GO:0043185] (molecular function) Also known as: VEGF receptor 3 binding, VEGFR 3 binding, fms-like-tyrosine kinase (Flt)-4 binding Definition: Binding to a vascular endothelial growth factor receptor 3. Relationships: is a type of vascular endothelial growth factor receptor binding [GO:0005172] Sources: GOC:st